{
  "term_id": "UNKNOWN:0002",
  "gene_symbol": "CPXM1",
  "gene_name": "Probable carboxypeptidase X1",
  "gene": "UniProtKB:Q96SM3",
  "term_label": "Unknown biological process"
}